type 5 melanocortin receptor binding [GO:0031783] (molecular function) Relationships: is a type of melanocortin receptor binding [GO:0031779] Sources: GOC:mah, GOC:nln Also known as: type 5 melanocortin receptor ligand Definition: Binding to a type 5 melanocortin receptor.